cytoskeletal motor activity [GO:0003774] (molecular function) Subtypes: GO:0000146, microtubule motor activity [GO:0003777], GO:0061791, proton motive force-driven motor activity [GO:0140605] Also known as: motor activity References: PMID:11242086, PMID:29716949 Sources: GOC:mah, GOC:vw Definition: Generation of force resulting in movement, for example along a microfilament or microtubule, or in torque resulting in membrane scission or rotation of a flagellum. The energy required is obtained either from the hydrolysis of a nucleoside triphosphate or by an electrochemical proton gradient (proton-motive force). Regulation: regulated by GO:0140659; RO_0002213 by cytoskeletal motor activator activity [GO:0140660]; negatively regulated by cytoskeletal motor inhibitor activity [GO:0140661] Relationships: is a type of molecular_function [GO:0003674]